{
  "gene_name": "C-type lectin domain family 19 member A",
  "gene": "UniProtKB:Q6UXS0",
  "gene_symbol": "CLEC19A",
  "term_id": "UNKNOWN:0002",
  "term_label": "Unknown biological process"
}